{
  "term_id": "GO:0086089",
  "gene_name": "Potassium voltage-gated channel subfamily KQT member 1",
  "term_label": "voltage-gated potassium channel activity involved in atrial cardiac muscle cell action potential repolarization",
  "gene": "UniProtKB:P51787",
  "gene_symbol": "KCNQ1"
}